{
  "gene_name": "Transmembrane emp24 domain-containing protein 3",
  "gene": "UniProtKB:Q9Y3Q3",
  "gene_symbol": "TMED3",
  "term_label": "COPI vesicle coat",
  "term_id": "GO:0030126"
}